{
  "gene_symbol": "DKK1",
  "gene_name": "Dickkopf-related protein 1",
  "gene": "UniProtKB:O94907",
  "term_label": "co-receptor binding",
  "term_id": "GO:0039706"
}